{
  "term_label": "RZZ complex",
  "term_id": "GO:1990423",
  "gene": "UniProtKB:O43264",
  "gene_symbol": "ZW10",
  "gene_name": "Centromere_kinetochore protein zw10 homolog"
}